calprotectin complex [GO:1990660] (cellular component) Note: An example of this is S100A9 in human (UniProt symbol P06702) in PMID:25417112 (inferred from direct assay). Also known as: calprotectin heterodimer Relationships: is a type of protein-containing complex [GO:0032991] References: PMID:25417112 Sources: GOC:bhm Definition: A protein complex composed of S100A8 and S100A9 and capable of limiting Mn(2+) and Zn(2+) availability at sites of infection. Also binds Ca(2+). Expressed and released by neutrophils and epithelial cells, it exhibits broad-spectrum antimicrobial activity attributed to its metal-binding properties. Endogenous ligand of toll-like receptor 4 (TLR4) and of the receptor for advanced glycation end products (RAGE) initiating signal transduction through NF-kappa-B pathways.